{
  "term_id": "GO:0000978",
  "gene_symbol": "ZNF664",
  "term_label": "RNA polymerase II cis-regulatory region sequence-specific DNA binding",
  "gene": "UniProtKB:Q8N3J9",
  "gene_name": "Zinc finger protein 664"
}